negative regulation of receptor clustering [GO:1903910] (biological process) References: PMID:23575248 Sources: GOC:TermGenie, GOC:als, GO_REF:0000058 Subtypes: GO:1904394, negative regulation of AMPA glutamate receptor clustering [GO:1904718] Definition: Any process that stops, prevents or reduces the frequency, rate or extent of receptor clustering. Also known as: down regulation of receptor clustering, down-regulation of receptor clustering, downregulation of receptor clustering, inhibition of receptor clustering Relationships: is a type of GO:1903909; is a type of GO:1905476; negatively regulates receptor clustering [GO:0043113]